{
  "term_id": "GO:0060074",
  "gene_name": "Seizure 6-like protein",
  "gene": "UniProtKB:Q9BYH1",
  "term_label": "synapse maturation",
  "gene_symbol": "SEZ6L"
}